{
  "gene_symbol": "DDHD2",
  "term_label": "triacylglycerol lipase activity",
  "gene": "UniProtKB:O94830",
  "gene_name": "Phospholipase DDHD2",
  "term_id": "GO:0004806"
}